organellar chromatophore inner membrane [GO:0070113] (cellular component) Also known as: Paulinella-type chromatophore inner membrane Relationships: is a type of organellar chromatophore membrane [GO:0070112] Sources: GOC:mah Definition: The inner, i.e. lumen-facing, of the two lipid bilayers surrounding an organellar chromatophore.